{
  "term_id": "GO:0015990",
  "term_label": "electron transport coupled proton transport",
  "gene": "UniProtKB:P03905",
  "gene_name": "NADH-ubiquinone oxidoreductase chain 4",
  "gene_symbol": "MT-ND4"
}